{
  "gene_symbol": "MAD2L1",
  "gene_name": "Mitotic spindle assembly checkpoint protein MAD2A",
  "term_label": "kinetochore",
  "gene": "UniProtKB:Q13257",
  "term_id": "GO:0000776"
}